{
  "gene": "UniProtKB:Q15797",
  "gene_symbol": "SMAD1",
  "term_label": "cell differentiation",
  "gene_name": "Mothers against decapentaplegic homolog 1",
  "term_id": "GO:0030154"
}